{
  "term_label": "actin polymerization or depolymerization",
  "term_id": "GO:0008154",
  "gene_symbol": "AVIL",
  "gene_name": "Advillin",
  "gene": "UniProtKB:O75366"
}